{
  "gene_symbol": "UBXN2B",
  "gene": "UniProtKB:Q14CS0",
  "term_id": "GO:0005829",
  "term_label": "cytosol",
  "gene_name": "UBX domain-containing protein 2B"
}